{
  "term_id": "GO:0044325",
  "gene_symbol": "KCNE4",
  "gene_name": "Potassium voltage-gated channel subfamily E member 4",
  "term_label": "transmembrane transporter binding",
  "gene": "UniProtKB:Q8WWG9"
}